{
  "gene": "UniProtKB:Q9BXM7",
  "gene_name": "Serine_threonine-protein kinase PINK1, mitochondrial",
  "term_label": "protein serine/threonine kinase activity",
  "term_id": "GO:0004674",
  "gene_symbol": "PINK1"
}